{
  "term_label": "embryonic skeletal system morphogenesis",
  "gene_symbol": "HOXC4",
  "gene": "UniProtKB:P09017",
  "gene_name": "Homeobox protein Hox-C4",
  "term_id": "GO:0048704"
}